carbon catabolite activation of transcription [GO:0045991] (biological process) Definition: A transcription regulation process in which the presence of one carbon source leads to an increase in the frequency, rate, or extent of transcription of specific genes involved in the metabolism of other carbon sources. References: PMID:10559153 Sources: GOC:mah Also known as: positive regulation of transcription by carbon catabolites Relationships: is a type of positive regulation of DNA-templated transcription [GO:0045893]; is a type of carbon catabolite regulation of transcription [GO:0045990] Subtypes: positive regulation of transcription by galactose [GO:0000411], GO:0000436, positive regulation of transcription by glucose [GO:0046016]